regulation of dendritic spine maintenance [GO:1902950] (biological process) Subtypes: GO:1902951, positive regulation of dendritic spine maintenance [GO:1902952] Definition: Any process that modulates the frequency, rate or extent of dendritic spine maintenance. References: PMID:24328732 Sources: GOC:TermGenie, GOC:sjp, GO_REF:0000058 Relationships: is a type of GO:0099175; is a type of regulation of plasma membrane bounded cell projection organization [GO:0120035]; regulates dendritic spine maintenance [GO:0097062]